{
  "term_id": "GO:0000978",
  "term_label": "RNA polymerase II cis-regulatory region sequence-specific DNA binding",
  "gene": "UniProtKB:Q0D2J5",
  "gene_symbol": "ZNF763",
  "gene_name": "Zinc finger protein 763"
}